rRNA import into mitochondrion [GO:0035928] (biological process) Relationships: is a type of GO:0035927; is a type of GO:0051029 Also known as: cytoplasmic rRNA import into mitochondrion, nuclear-encoded rRNA import into mitochondrion Definition: The process in which a rRNA, ribosomal ribonucleic acid, transported from the cytosol into the mitochondrial matrix. References: PMID:20691904 Sources: GOC:ans